{
  "gene_symbol": "RPL23A",
  "gene_name": "Large ribosomal subunit protein uL23",
  "term_id": "UNKNOWN:0002",
  "term_label": "Unknown biological process",
  "gene": "UniProtKB:P62750"
}